{
  "gene_name": "Glutamate receptor 4",
  "term_label": "transmitter-gated monoatomic ion channel activity involved in regulation of postsynaptic membrane potential",
  "gene_symbol": "GRIA4",
  "term_id": "GO:1904315",
  "gene": "UniProtKB:P48058"
}